{
  "gene_symbol": "MFN2",
  "gene_name": "Mitofusin-2",
  "gene": "UniProtKB:O95140",
  "term_id": "GO:0008053",
  "term_label": "mitochondrial fusion"
}